transcription ternary complex disassembly [GO:0001118] (BP) Definition: The disaggregation of a transcription ternary complex, composed of RNA polymerase, template DNA, and an RNA transcript, into its constituent components. Also known as: transcription protein-DNA-RNA complex disassembly Sources: GOC:txnOH Relationships: is a type of protein-DNA-RNA complex disassembly [GO:0001117]; BFO_0000050 DNA-templated transcription termination [GO:0006353]